phosphatidylethanolamine:Kdo2-lipid A phosphoethanolamine transferase activity [GO:0043838] (molecular function) Also known as: phosphoethanolamine transferase, EptB Definition: Catalysis of the reaction: Kdo2-lipid A + phosphatidylethanolamine = phosphoethanolamine-Kdo2-lipid A + diacylglycerol. Relationships: is a type of phosphotransferase activity, for other substituted phosphate groups [GO:0016780] References: PMID:15795227 Note: Note that Kdo is an abbreviation for 3-deoxy-D-manno-oct-2-ulosonic acid.